{
  "gene_symbol": "OR5AL1",
  "gene": "UniProtKB:P0C617",
  "term_label": "Unknown biological process",
  "gene_name": "Olfactory receptor 5AL1",
  "term_id": "UNKNOWN:0002"
}